{
  "gene": "UniProtKB:P25100",
  "term_id": "GO:0007200",
  "term_label": "phospholipase C-activating G protein-coupled receptor signaling pathway",
  "gene_symbol": "ADRA1D",
  "gene_name": "Alpha-1D adrenergic receptor"
}